{
  "gene_symbol": "SOX1",
  "gene_name": "Transcription factor SOX-1",
  "term_id": "GO:0007420",
  "term_label": "brain development",
  "gene": "UniProtKB:O00570"
}